{
  "gene_name": "Protein moonraker",
  "term_label": "centriolar satellite",
  "gene_symbol": "KIAA0753",
  "gene": "UniProtKB:Q2KHM9",
  "term_id": "GO:0034451"
}